{
  "term_label": "endosome",
  "gene_name": "Rab GTPase-binding effector protein 1",
  "gene_symbol": "RABEP1",
  "gene": "UniProtKB:Q15276",
  "term_id": "GO:0005768"
}